protein targeting to mitochondrion [GO:0006626] (biological process) Regulation: regulated by regulation of protein targeting to mitochondrion [GO:1903214]; negatively regulated by negative regulation of protein targeting to mitochondrion [GO:1903215]; positively regulated by positive regulation of protein targeting to mitochondrion [GO:1903955] Definition: The process of directing proteins towards and into the mitochondrion, usually mediated by mitochondrial proteins that recognize signals contained within the imported protein. Also known as: protein import into mitochondrion, protein targeting to mitochondria, protein-mitochondrial targeting, mitochondrial protein import, mitochondrial translocation Sources: GOC:mcc, ISBN:0716731363 Relationships: is a type of protein targeting [GO:0006605]; is a type of establishment of protein localization to mitochondrion [GO:0072655]